negative regulation of centrosome duplication [GO:0010826] (biological process) Definition: Any process that decreases the frequency, rate or extent of centrosome duplication. Centrosome duplication is the replication of a centrosome, a structure comprised of a pair of centrioles and peri-centriolar material from which a microtubule spindle apparatus is organized. Sources: GOC:dph, GOC:tb Relationships: is_a regulation of centrosome duplication [GO:0010824]; is a type of negative regulation of centrosome cycle [GO:0046606]; negatively regulates GO:0051298 Subtypes: negative regulation of centriole replication [GO:0046600]